{
  "gene_name": "Cytochrome P450 11B2, mitochondrial",
  "term_id": "GO:0006704",
  "gene": "UniProtKB:P19099",
  "term_label": "glucocorticoid biosynthetic process",
  "gene_symbol": "CYP11B2"
}